{
  "term_id": "GO:0098700",
  "gene_name": "Vesicular glutamate transporter 2",
  "term_label": "neurotransmitter loading into synaptic vesicle",
  "gene": "UniProtKB:Q9P2U8",
  "gene_symbol": "SLC17A6"
}